monoterpenol O-acetyltransferase activity [GO:0050107] (molecular function) Sources: EC:2.3.1.69, MetaCyc:MONOTERPENOL-O-ACETYLTRANSFERASE-RXN Also known as: menthol transacetylase activity, acetyl-CoA:monoterpenol O-acetyltransferase activity Definition: Catalysis of the reaction: acetyl-CoA + a monoterpenol = CoA + a monoterpenol acetate ester. Relationships: is a type of O-acetyltransferase activity [GO:0016413]